positive regulation of gene expression [GO:0010628] (biological process) Definition: Any process that increases the frequency, rate or extent of gene expression. Gene expression is the process in which a gene's coding sequence is converted into a mature gene product (protein or RNA). Relationships: is_a GO:0010468; is a type of positive regulation of macromolecule biosynthetic process [GO:0010557]; positively regulates gene expression [GO:0010467] Subtypes: positive regulation of cytokine production [GO:0001819], positive regulation of production of molecular mediator of immune response [GO:0002702], negative regulation of heterochromatin formation [GO:0031452], transcription antitermination [GO:0031564], positive regulation of RNA splicing [GO:0033120], GO:0045727, negative regulation of post-transcriptional gene silencing [GO:0060149], negative regulation of gene silencing by regulatory ncRNA [GO:0060967], GO:0140668, zygotic genome activation [GO:0141064], positive regulation of gene expression, epigenetic [GO:0141137], negative regulation of mRNA catabolic process [GO:1902373], positive regulation of snoRNA processing [GO:1902798], positive regulation of protein maturation [GO:1903319], GO:1903800, positive regulation of 3'-UTR-mediated mRNA stabilization [GO:1905870], positive regulation of tRNA processing [GO:2000237] Sources: GOC:txnOH-2018